{
  "gene_name": "TRPM8 channel-associated factor 2",
  "term_id": "GO:0005886",
  "term_label": "plasma membrane",
  "gene": "UniProtKB:A6NFQ2",
  "gene_symbol": "TCAF2"
}